{
  "gene": "UniProtKB:Q9NZ53",
  "gene_symbol": "PODXL2",
  "gene_name": "Podocalyxin-like protein 2",
  "term_id": "UNKNOWN:0003",
  "term_label": "Unknown cellular component"
}